{
  "gene_symbol": "DEFB133",
  "term_label": "extracellular space",
  "gene_name": "Beta-defensin 133",
  "gene": "UniProtKB:Q30KQ1",
  "term_id": "GO:0005615"
}